{
  "gene_name": "Zinc finger protein 773",
  "term_label": "DNA-binding transcription factor activity, RNA polymerase II-specific",
  "gene": "UniProtKB:Q6PK81",
  "gene_symbol": "ZNF773",
  "term_id": "GO:0000981"
}